{
  "term_label": "protein processing involved in protein targeting to mitochondrion",
  "gene": "UniProtKB:Q96LU5",
  "gene_name": "Mitochondrial inner membrane protease subunit 1",
  "gene_symbol": "IMMP1L",
  "term_id": "GO:0006627"
}